response to decane [GO:1902782] (biological process) Definition: Any process that results in a change in state or activity of a cell or an organism (in terms of movement, secretion, enzyme production, gene expression, etc.) as a result of a decane stimulus. References: PMID:23826995 Sources: GOC:TermGenie, GOC:mengo_curators, GO_REF:0000071 Subtypes: cellular response to decane [GO:1902783] Relationships: is a type of response to alkane [GO:1902778]